{
  "gene_name": "Breast cancer anti-estrogen resistance protein 3",
  "gene": "UniProtKB:O75815",
  "term_label": "positive regulation of MAPK cascade",
  "term_id": "GO:0043410",
  "gene_symbol": "BCAR3"
}